{
  "gene_name": "Glycosyltransferase-like domain-containing protein 1",
  "term_label": "cytoplasm",
  "gene_symbol": "GTDC1",
  "term_id": "GO:0005737",
  "gene": "UniProtKB:Q4AE62"
}